fruit valve development [GO:1990059] (biological process) Definition: The process whose specific outcome is the progression of the fruit valve over time, from its formation to the mature structure. The fruit valve is a part of a fruit that splits apart when the fruit dehisces. Relationships: is_a GO:0009791; is a type of GO:0048856; is part of GO:0010154 References: PMID:23133401 Sources: PO:0000033